meiotic metaphase I [GO:0007132] (biological process) Note: Note that this term should not be used for direct annotation. If you are trying to make an annotation to x phase, it is likely that the correct annotation is 'regulation of x/y phase transition' or to a process which occurs during the reported phase (i.e mitotic DNA replication for mitotic S-phase). To capture the phase when a specific location or process is observed, the phase term can be used in an annotation extension (PMID:24885854) applied to a cellular component term (with the relation exists_during) or a biological process term (with the relation happens_during). Sources: GOC:mtg_cell_cycle Relationships: is a type of meiosis I cell cycle phase [GO:0098764]; is part of metaphase [GO:0051323]; is part of meiotic M phase [GO:0051327] Definition: The cell cycle phase, following prophase I, during which chromosomes become aligned on the equatorial plate of the cell as part of meiosis I.